{
  "term_id": "GO:0060291",
  "gene_name": "Sodium_potassium_calcium exchanger 1",
  "term_label": "long-term synaptic potentiation",
  "gene": "UniProtKB:O60721",
  "gene_symbol": "SLC24A1"
}